{
  "gene_symbol": "SAT2",
  "gene": "UniProtKB:Q96F10",
  "term_label": "Unknown biological process",
  "term_id": "UNKNOWN:0002",
  "gene_name": "Thialysine N-epsilon-acetyltransferase"
}